{
  "term_id": "GO:2000145",
  "gene_name": "Inactive tyrosine-protein kinase PEAK1",
  "gene_symbol": "PEAK1",
  "gene": "UniProtKB:Q9H792",
  "term_label": "regulation of cell motility"
}